{
  "gene": "UniProtKB:Q9Y5X4",
  "gene_name": "Photoreceptor-specific nuclear receptor",
  "term_label": "RNA polymerase II cis-regulatory region sequence-specific DNA binding",
  "term_id": "GO:0000978",
  "gene_symbol": "NR2E3"
}